positive regulation of siderophore biosynthetic process [GO:1900706] (biological process) Definition: Any process that activates or increases the frequency, rate or extent of siderophore biosynthetic process. Sources: GOC:TermGenie, GOC:di Also known as: activation of siderophore anabolism, activation of siderophore biosynthesis, activation of siderophore formation, activation of siderophore synthesis, positive regulation of siderophore anabolism, positive regulation of siderophore biosynthesis, positive regulation of siderophore formation, positive regulation of siderophore synthesis, up regulation of siderophore anabolism, up regulation of siderophore biosynthesis, up regulation of siderophore biosynthetic process, up regulation of siderophore formation, up regulation of siderophore synthesis, up-regulation of siderophore anabolism, up-regulation of siderophore biosynthesis, up-regulation of siderophore biosynthetic process, up-regulation of siderophore formation, up-regulation of siderophore synthesis, upregulation of siderophore anabolism, upregulation of siderophore biosynthesis, upregulation of siderophore biosynthetic process, upregulation of siderophore formation, upregulation of siderophore synthesis, activation of siderochrome biosynthesis, activation of siderochrome biosynthetic process, activation of siderophore biosynthetic process, activation of siderophore biosynthetic process, peptide formation, activation of siderophore biosynthetic process, peptide modification, positive regulation of siderochrome biosynthesis, positive regulation of siderochrome biosynthetic process, positive regulation of siderophore biosynthetic process, peptide formation, positive regulation of siderophore biosynthetic process, peptide modification, up regulation of siderochrome biosynthesis, up regulation of siderochrome biosynthetic process, up regulation of siderophore biosynthetic process, peptide formation, up regulation of siderophore biosynthetic process, peptide modification, up-regulation of siderochrome biosynthesis, up-regulation of siderochrome biosynthetic process, up-regulation of siderophore biosynthetic process, peptide formation, up-regulation of siderophore biosynthetic process, peptide modification, upregulation of siderochrome biosynthesis, upregulation of siderochrome biosynthetic process, upregulation of siderophore biosynthetic process, peptide formation, upregulation of siderophore biosynthetic process, peptide modification Relationships: is_a positive regulation of secondary metabolite biosynthetic process [GO:1900378]; is a type of regulation of siderophore biosynthetic process [GO:1900704]; positively regulates siderophore biosynthetic process [GO:0019290] Subtypes: GO:1905570